{
  "gene_name": "Leukocyte cell-derived chemotaxin 1",
  "term_label": "negative regulation of angiogenesis",
  "term_id": "GO:0016525",
  "gene": "UniProtKB:O75829",
  "gene_symbol": "CNMD"
}